{
  "gene_symbol": "EXOSC8",
  "gene_name": "Exosome complex component RRP43",
  "gene": "UniProtKB:Q96B26",
  "term_label": "U4 snRNA 3'-end processing",
  "term_id": "GO:0034475"
}